{
  "gene_name": "Fibroblast growth factor 4",
  "term_label": "regulation of cell migration",
  "term_id": "GO:0030334",
  "gene": "UniProtKB:P08620",
  "gene_symbol": "FGF4"
}